{
  "term_id": "GO:0071549",
  "gene_symbol": "PCK1",
  "gene_name": "Phosphoenolpyruvate carboxykinase, cytosolic [GTP]",
  "gene": "UniProtKB:P35558",
  "term_label": "cellular response to dexamethasone stimulus"
}